{
  "gene": "UniProtKB:Q86TS9",
  "term_label": "translation",
  "gene_name": "Large ribosomal subunit protein mL52",
  "term_id": "GO:0006412",
  "gene_symbol": "MRPL52"
}